{
  "term_label": "mechanosensitive monoatomic ion channel activity",
  "gene_symbol": "TMC6",
  "gene_name": "Transmembrane channel-like protein 6",
  "term_id": "GO:0008381",
  "gene": "UniProtKB:Q7Z403"
}